copal-8-ol diphosphate synthase activity [GO:0102161] (MF) Relationships: is a type of hydro-lyase activity [GO:0016836] Sources: EC:4.2.1.133, GOC:pz Definition: Catalysis of the reaction: copal-8-ol diphosphate = 2-trans,6-trans,10-trans-geranylgeranyl diphosphate + H2O.